{
  "gene_name": "Dynamin-1",
  "term_label": "synapse",
  "term_id": "GO:0045202",
  "gene_symbol": "DNM1",
  "gene": "UniProtKB:Q05193"
}